late stripe melanocyte differentiation [GO:0050934] (BP) Definition: The process in which a relatively unspecialized cell acquires the specialized features of a late stripe melanocyte (LSM). In zebrafish, LSMs develop during the second phase (3-4 weeks of development) of the larva-to-adult transition (2-4 weeks of development). References: PMID:11858836 Also known as: late stripe melanocyte cell differentiation, late stripe melanophore differentiation Relationships: is a type of melanocyte differentiation [GO:0030318] Regulation: regulated by regulation of late stripe melanocyte differentiation [GO:0050940]; negatively regulated by GO:0050949; positively regulated by GO:0050950